{
  "gene_name": "Major intrinsically disordered NOTCH2-binding receptor 1-like",
  "gene": "UniProtKB:P59773",
  "term_label": "Unknown biological process",
  "term_id": "UNKNOWN:0002",
  "gene_symbol": "MINAR2"
}